{
  "gene": "UniProtKB:P78410",
  "term_id": "GO:0001817",
  "gene_name": "Butyrophilin subfamily 3 member A2",
  "term_label": "regulation of cytokine production",
  "gene_symbol": "BTN3A2"
}